{
  "gene_name": "Laminin subunit alpha-5",
  "term_id": "GO:0034446",
  "gene": "UniProtKB:O15230",
  "gene_symbol": "LAMA5",
  "term_label": "substrate adhesion-dependent cell spreading"
}